{
  "gene_name": "EF-hand calcium-binding domain-containing protein 13",
  "term_label": "Unknown biological process",
  "gene": "UniProtKB:Q8IY85",
  "gene_symbol": "EFCAB13",
  "term_id": "UNKNOWN:0002"
}